{
  "term_label": "DNA-binding transcription factor activity, RNA polymerase II-specific",
  "gene_symbol": "HOXA7",
  "gene": "UniProtKB:P31268",
  "term_id": "GO:0000981",
  "gene_name": "Homeobox protein Hox-A7"
}